{
  "gene": "UniProtKB:Q03164",
  "gene_name": "Histone-lysine N-methyltransferase 2A",
  "term_id": "GO:0042800",
  "term_label": "histone H3K4 methyltransferase activity",
  "gene_symbol": "KMT2A"
}